{
  "gene": "UniProtKB:Q67FW5",
  "term_label": "Unknown cellular component",
  "gene_symbol": "B3GNTL1",
  "term_id": "UNKNOWN:0003",
  "gene_name": "UDP-GlcNAc:betaGal beta-1,3-N-acetylglucosaminyltransferase-like protein 1"
}